{
  "term_label": "detection of mechanical stimulus",
  "gene_symbol": "PKDREJ",
  "term_id": "GO:0050982",
  "gene_name": "Polycystin family receptor for egg jelly",
  "gene": "UniProtKB:Q9NTG1"
}